{
  "gene": "UniProtKB:Q9UHF5",
  "term_id": "UNKNOWN:0003",
  "gene_name": "Interleukin-17B",
  "term_label": "Unknown cellular component",
  "gene_symbol": "IL17B"
}